{
  "term_label": "plasma membrane",
  "term_id": "GO:0005886",
  "gene": "UniProtKB:Q8N0X7",
  "gene_name": "Spartin",
  "gene_symbol": "SPART"
}